{
  "term_id": "UNKNOWN:0001",
  "term_label": "Unknown molecular function",
  "gene_name": "A-kinase-interacting protein 1",
  "gene": "UniProtKB:Q9NQ31",
  "gene_symbol": "AKIP1"
}